protocadherin-alpha-v7-protocadherin-gamma-a1 complex [GO:0071188] (cellular component) Definition: A protein complex that contains the cell adhesion molecules protocadherin-alpha-v7 and protocadherin-gamma-a1, and is involved in the regulation of protein localization to the plasma membrane. Also known as: Pcdha7-Pcdhga1 complex References: PMID:15347688 Relationships: is a type of GO:0071183